{
  "gene_symbol": "CCDC15",
  "term_id": "GO:0005813",
  "term_label": "centrosome",
  "gene": "UniProtKB:Q0P6D6",
  "gene_name": "Coiled-coil domain-containing protein 15"
}